regulation of translation in response to stress [GO:0043555] (biological process) Sources: GOC:jl Relationships: is_a GO:0006417; is part of cellular response to stress [GO:0033554] Subtypes: negative regulation of translation in response to stress [GO:0032055], positive regulation of translation in response to stress [GO:0032056], regulation of translation in response to endoplasmic reticulum stress [GO:0036490], regulation of translation in response to osmotic stress [GO:0043557], regulation of translational initiation in response to stress [GO:0043558], regulation of cytoplasmic translation in response to stress [GO:1990497] Definition: Modulation of the frequency, rate or extent of translation as a result of a stimulus indicating the organism is under stress. The stress is usually, but not necessarily, exogenous (e.g. temperature, humidity, ionizing radiation). Also known as: translational stress response